{
  "gene_symbol": "PTPRN2",
  "gene": "UniProtKB:Q92932",
  "gene_name": "Receptor-type tyrosine-protein phosphatase N2",
  "term_label": "regulation of secretion",
  "term_id": "GO:0051046"
}